{
  "gene": "UniProtKB:Q5T4T1",
  "term_label": "plasma membrane",
  "gene_name": "Transmembrane protein 170B",
  "term_id": "GO:0005886",
  "gene_symbol": "TMEM170B"
}